{
  "gene_symbol": "RBM42",
  "term_label": "mRNA binding",
  "term_id": "GO:0003729",
  "gene_name": "RNA-binding protein 42",
  "gene": "UniProtKB:Q9BTD8"
}